{
  "term_id": "GO:0050911",
  "term_label": "detection of chemical stimulus involved in sensory perception of smell",
  "gene_symbol": "OR2Z1",
  "gene_name": "Olfactory receptor 2Z1",
  "gene": "UniProtKB:Q8NG97"
}